{
  "gene_symbol": "ESPL1",
  "term_label": "centrosome",
  "gene_name": "Separin",
  "term_id": "GO:0005813",
  "gene": "UniProtKB:Q14674"
}